{
  "gene_name": "Putative uncharacterized protein PNAS-138",
  "term_label": "Unknown molecular function",
  "gene": "UniProtKB:Q9BZS9",
  "gene_symbol": "PNAS-138",
  "term_id": "UNKNOWN:0001"
}